{
  "gene_symbol": "PRDX2",
  "gene": "UniProtKB:P32119",
  "term_id": "GO:0019430",
  "gene_name": "Peroxiredoxin-2",
  "term_label": "removal of superoxide radicals"
}